{
  "gene_symbol": "PI3",
  "term_label": "serine-type endopeptidase inhibitor activity",
  "term_id": "GO:0004867",
  "gene_name": "Elafin",
  "gene": "UniProtKB:P19957"
}